estrous cycle [GO:0044849] (biological process) Definition: A type of ovulation cycle, which occurs in most mammalian therian females, where the endometrium is resorbed if pregnancy does not occur. Relationships: is a type of ovulation cycle [GO:0042698] Sources: GOC:jl, Wikipedia:Estrous_cycle